{
  "gene": "UniProtKB:Q6ZU80",
  "term_id": "UNKNOWN:0002",
  "gene_symbol": "CEP128",
  "gene_name": "Centrosomal protein of 128 kDa",
  "term_label": "Unknown biological process"
}